{
  "term_id": "GO:0006354",
  "term_label": "DNA-templated transcription elongation",
  "gene_name": "AF4_FMR2 family member 2",
  "gene": "UniProtKB:P51816",
  "gene_symbol": "AFF2"
}